leading edge of dendritic growth cone [GO:0061917] (cellular component) References: PMID:16098134 Definition: That part of the dendritic growth cone which represents the distal part of the structure. Relationships: is a type of growth cone leading edge [GO:0061850]; is part of dendritic growth cone [GO:0044294] Also known as: dendritic growth cone leading edge, distal tip of dendritic growth cone